{
  "gene_name": "DDB1- and CUL4-associated factor 10",
  "gene": "UniProtKB:Q5QP82",
  "term_label": "Unknown molecular function",
  "gene_symbol": "DCAF10",
  "term_id": "UNKNOWN:0001"
}